sialate:monoatomic cation symporter activity [GO:0015306] (molecular function) Definition: Enables the transfer of a solute or solutes from one side of a membrane to the other according to the reaction: sialate(out) + cation(out) = sialate(in) + cation(in). Sources: TC:2.A.1.14.10 Relationships: is a type of sialic acid transmembrane transporter activity [GO:0015136]; is a type of GO:0015294; is_a GO:0042887; is a type of carboxylic acid transmembrane transporter activity [GO:0046943] Also known as: sialate transporter activity, sialate:cation symporter activity, cation/sialate symporter activity, cation:sialate symporter activity, sialate/cation symporter activity